{
  "term_label": "nucleus",
  "gene_name": "Small ribosomal subunit protein RACK1",
  "gene": "UniProtKB:P63244",
  "term_id": "GO:0005634",
  "gene_symbol": "RACK1"
}